{
  "gene_symbol": "ZNF280C",
  "term_id": "GO:0000978",
  "gene": "UniProtKB:Q8ND82",
  "gene_name": "Zinc finger protein 280C",
  "term_label": "RNA polymerase II cis-regulatory region sequence-specific DNA binding"
}